{
  "term_label": "potassium channel regulator activity",
  "gene_symbol": "KCNE3",
  "gene": "UniProtKB:Q9Y6H6",
  "gene_name": "Potassium voltage-gated channel subfamily E member 3",
  "term_id": "GO:0015459"
}